positive regulation of cell chemotaxis to fibroblast growth factor [GO:1904849] (biological process) Definition: Any process that activates or increases the frequency, rate or extent of cell chemotaxis to fibroblast growth factor. References: PMID:23233752 Sources: GOC:BHF, GOC:BHF_miRNA, GOC:TermGenie, GOC:rph, GO_REF:0000058 Also known as: up regulation of cell chemotaxis to fibroblast growth factor, up-regulation of cell chemotaxis to fibroblast growth factor, upregulation of cell chemotaxis to fibroblast growth factor, activation of cell chemotaxis to fibroblast growth factor Relationships: is a type of GO:0030335; is a type of GO:0050921; is a type of regulation of cell chemotaxis to fibroblast growth factor [GO:1904847]; positively regulates cell chemotaxis to fibroblast growth factor [GO:0035766] Subtypes: positive regulation of endothelial cell chemotaxis to fibroblast growth factor [GO:2000546]